{
  "gene_name": "Solute carrier family 12 member 2",
  "term_label": "sodium ion transmembrane transport",
  "gene_symbol": "SLC12A2",
  "term_id": "GO:0035725",
  "gene": "UniProtKB:P55011"
}